{
  "gene": "UniProtKB:Q96MD7",
  "term_id": "UNKNOWN:0002",
  "gene_symbol": "C9orf85",
  "gene_name": "Uncharacterized protein C9orf85",
  "term_label": "Unknown biological process"
}